negative regulation of establishment of protein localization to mitochondrion [GO:1903748] (biological process) Also known as: down regulation of establishment of protein localisation to mitochondrion, down regulation of establishment of protein localization in mitochondrion, down regulation of establishment of protein localization to mitochondrion, down-regulation of establishment of protein localisation to mitochondrion, down-regulation of establishment of protein localization in mitochondrion, down-regulation of establishment of protein localization to mitochondrion, downregulation of establishment of protein localisation to mitochondrion, downregulation of establishment of protein localization in mitochondrion, downregulation of establishment of protein localization to mitochondrion, negative regulation of establishment of protein localisation to mitochondrion, negative regulation of establishment of protein localization in mitochondrion, inhibition of establishment of protein localisation to mitochondrion, inhibition of establishment of protein localization in mitochondrion, inhibition of establishment of protein localization to mitochondrion Subtypes: negative regulation of protein targeting to mitochondrion [GO:1903215] Definition: Any process that stops, prevents or reduces the frequency, rate or extent of establishment of protein localization to mitochondrion. References: PMID:16857185 Sources: GOC:TermGenie, GO_REF:0000058 Relationships: is_a regulation of establishment of protein localization to mitochondrion [GO:1903747]; is a type of negative regulation of establishment of protein localization [GO:1904950]; negatively regulates establishment of protein localization to mitochondrion [GO:0072655]